galactonolactone dehydrogenase activity [GO:0016633] (molecular function) Also known as: L-galactono-1,4-lactone dehydrogenase activity, GLDHase activity, GLDase activity, L-galactono-1,4-lactone:ferricytochrome-c oxidoreductase activity, L-galactono-gamma-lactone dehydrogenase activity, L-galactono-gamma-lactone:ferricytochrome-c oxidoreductase activity, L-galactonolactone dehydrogenase activity Relationships: is a type of oxidoreductase activity, acting on the CH-CH group of donors, cytochrome as acceptor [GO:0016632] Sources: EC:1.3.2.3 Definition: Catalysis of the reaction: L-galactono-1,4-lactone + 2 ferricytochrome c = L-ascorbate + 2 ferrocytochrome c.